ethanolamine oxidase activity [GO:0047883] (molecular function) Sources: RHEA:18581 Also known as: ethanolamine:oxygen oxidoreductase (deaminating) Definition: Catalysis of the reaction: ethanolamine + H2O + O2 = glycolaldehyde + NH3 + H2O2. Relationships: is a type of aliphatic amine oxidase activity [GO:0052595]